negative regulation of intracellular cholesterol transport [GO:0032384] (biological process) Sources: GOC:mah Definition: Any process that stops, prevents, or reduces the frequency, rate or extent of the directed movement of cholesterol within cells. Also known as: down regulation of intracellular cholesterol transport, down-regulation of intracellular cholesterol transport, downregulation of intracellular cholesterol transport, inhibition of intracellular cholesterol transport Subtypes: negative regulation of receptor-mediated endocytosis involved in cholesterol transport [GO:1905601] Relationships: is_a negative regulation of cholesterol transport [GO:0032375]; is a type of GO:0032381; is a type of regulation of intracellular cholesterol transport [GO:0032383]; negatively regulates intracellular cholesterol transport [GO:0032367]